{
  "gene_symbol": "CTSH",
  "gene": "UniProtKB:P09668",
  "gene_name": "Pro-cathepsin H",
  "term_id": "GO:0004197",
  "term_label": "cysteine-type endopeptidase activity"
}